{
  "gene_name": "EEF1A lysine methyltransferase 2",
  "gene_symbol": "EEF1AKMT2",
  "gene": "UniProtKB:Q5JPI9",
  "term_label": "Unknown biological process",
  "term_id": "UNKNOWN:0002"
}